mechanoreceptor activity [GO:0140897] (molecular function) References: PMID:23907979, PMID:34666001 Definition: Combining with a mechanical force and transmitting the signal from one side of the membrane to the other to initiate a change in cell activity or state as part of signal transduction. Relationships: is_a transmembrane signaling receptor activity [GO:0004888]